{
  "term_id": "GO:0034727",
  "term_label": "piecemeal microautophagy of the nucleus",
  "gene_symbol": "ATG9B",
  "gene_name": "Autophagy-related protein 9B",
  "gene": "UniProtKB:Q674R7"
}